{
  "gene_name": "Mucin-20",
  "term_id": "UNKNOWN:0001",
  "gene": "UniProtKB:Q8N307",
  "term_label": "Unknown molecular function",
  "gene_symbol": "MUC20"
}